{
  "gene_name": "Metal transporter CNNM4",
  "gene": "UniProtKB:Q6P4Q7",
  "term_label": "magnesium ion transport",
  "term_id": "GO:0015693",
  "gene_symbol": "CNNM4"
}